succinate transmembrane transporter activity [GO:0015141] (molecular function) Subtypes: succinate:fumarate antiporter activity [GO:0005469], GO:0015515, GO:0015516, succinate:proton symporter activity [GO:0097434] Relationships: is a type of GO:0005310; is a type of C4-dicarboxylate transmembrane transporter activity [GO:0015556]; is part of succinate transmembrane transport [GO:0071422] Sources: ISBN:0198506732 Definition: Enables the transfer of succinate, the dianion of ethane dicarboxylic acid, from one side of a membrane to the other. Also known as: dicarboxylate (succinate/fumarate/malate) antiporter activity